{
  "gene_symbol": "PANK1",
  "gene_name": "Pantothenate kinase 1",
  "term_id": "GO:0004594",
  "term_label": "pantothenate kinase activity",
  "gene": "UniProtKB:Q8TE04"
}